{
  "term_label": "protein serine/threonine kinase activity",
  "gene_symbol": "DCLK1",
  "term_id": "GO:0004674",
  "gene": "UniProtKB:O15075",
  "gene_name": "Serine_threonine-protein kinase DCLK1"
}